decoy receptor complex [GO:0140368] (CC) Definition: A receptor complex that recognizes, binds and sequesters a specific receptor ligand to prevent it from binding to its regular receptor. May be soluble or membrane bound. References: PMID:30621730, PMID:9168977 Sources: GOC:bhm Relationships: is a type of receptor complex [GO:0043235] Also known as: osteoclastogenesis inhibitory factor, osteoprotegerin complex